positive regulation of receptor signaling pathway via STAT [GO:1904894] (biological process) Definition: Any process that activates or increases the frequency, rate or extent of receptor signaling pathway via STAT. Relationships: is a type of GO:0009967; is a type of regulation of receptor signaling pathway via STAT [GO:1904892]; positively regulates cell surface receptor signaling pathway via STAT [GO:0097696] Subtypes: positive regulation of receptor signaling pathway via JAK-STAT [GO:0046427] References: PMID:24587195 Sources: GOC:TermGenie, GOC:rjd, GO_REF:0000058 Also known as: positive regulation of STAT signalling pathway, positive regulation of kinase activated-STAT cascade, positive regulation of kinase-STAT cascade, up regulation of STAT cascade, up regulation of STAT signalling pathway, up regulation of kinase activated-STAT cascade, up regulation of kinase-STAT cascade, up-regulation of STAT cascade, up-regulation of STAT signalling pathway, up-regulation of kinase activated-STAT cascade, up-regulation of kinase-STAT cascade, upregulation of STAT cascade, upregulation of STAT signalling pathway, upregulation of kinase activated-STAT cascade, upregulation of kinase-STAT cascade, activation of STAT cascade, activation of STAT signalling pathway, activation of kinase activated-STAT cascade, activation of kinase-STAT cascade